gene expression involved in extracellular matrix organization [GO:1901148] (biological process) Definition: Any gene expression that is involved in extracellular matrix organization. Gene expression includes both transcription to produce an RNA transcript, and the translation of that mRNA into protein. Protein maturation is included in gene expression when required to form an active form of a product from an inactive precursor form. References: PMID:18668558 Sources: GOC:TermGenie, GOC:pg Also known as: expression of extracellular matrix proteins, extracellular matrix protein production Relationships: is_a gene expression [GO:0010467]; is part of extracellular matrix organization [GO:0030198]